{
  "gene_name": "Neutrophil defensin 3",
  "gene_symbol": "DEFA3",
  "gene": "UniProtKB:P59666",
  "term_label": "antibacterial humoral response",
  "term_id": "GO:0019731"
}